positive regulation of glomerular metanephric mesangial cell proliferation [GO:0072303] (BP) Relationships: is a type of positive regulation of glomerular mesangial cell proliferation [GO:0072126]; is a type of regulation of metanephric glomerular mesangial cell proliferation [GO:0072301]; positively regulates metanephric glomerular mesangial cell proliferation involved in metanephros development [GO:0072262] Sources: GOC:mtg_kidney_jan10 Definition: Any process that increases the frequency, rate or extent of metanephric glomerular mesangial cell proliferation.